{
  "gene_name": "Olfactory receptor 8K1",
  "term_id": "UNKNOWN:0003",
  "gene_symbol": "OR8K1",
  "term_label": "Unknown cellular component",
  "gene": "UniProtKB:Q8NGG5"
}